{
  "term_id": "GO:0005030",
  "gene": "UniProtKB:P04629",
  "gene_name": "High affinity nerve growth factor receptor",
  "gene_symbol": "NTRK1",
  "term_label": "neurotrophin receptor activity"
}